{
  "gene": "UniProtKB:P13569",
  "gene_name": "Cystic fibrosis transmembrane conductance regulator",
  "term_label": "intracellularly ATP-gated chloride channel activity",
  "term_id": "GO:0005260",
  "gene_symbol": "CFTR"
}